{
  "gene_name": "BTB_POZ domain-containing adapter for CUL3-mediated RhoA degradation protein 2",
  "term_id": "GO:0004842",
  "gene_symbol": "TNFAIP1",
  "gene": "UniProtKB:Q13829",
  "term_label": "ubiquitin-protein transferase activity"
}